capsorubin biosynthetic process [GO:1901866] (biological process) Relationships: is a type of xanthophyll biosynthetic process [GO:0016123] Definition: The chemical reactions and pathways resulting in the formation of capsorubin. Sources: GOC:TermGenie, GOC:yaf, MetaCyc:PWY-5174, UniPathway:UPA00807 Also known as: capsorubin anabolism, capsorubin biosynthesis, capsorubin formation, capsorubin synthesis